positive regulation of protein export from nucleus in response to glucose starvation [GO:0036279] (biological process) References: PMID:3541942 Sources: GOC:al Definition: Any process that activates or increases the frequency, rate or extent of directed movement of proteins from the nucleus into the cytoplasm in response to deprivation of glucose. Relationships: is a type of cellular response to glucose starvation [GO:0042149]; is a type of GO:0046827